{
  "gene": "UniProtKB:P39060",
  "gene_symbol": "COL18A1",
  "gene_name": "Collagen alpha-1(XVIII) chain",
  "term_label": "angiogenesis",
  "term_id": "GO:0001525"
}